{
  "term_label": "Unknown molecular function",
  "gene": "UniProtKB:P02585",
  "gene_symbol": "TNNC2",
  "gene_name": "Troponin C, skeletal muscle",
  "term_id": "UNKNOWN:0001"
}